{
  "gene_name": "Calcitonin gene-related peptide type 1 receptor",
  "gene": "UniProtKB:Q16602",
  "term_label": "calcitonin gene-related peptide receptor activity",
  "gene_symbol": "CALCRL",
  "term_id": "GO:0001635"
}